{
  "term_label": "sodium:proton antiporter activity",
  "gene_name": "Sodium_hydrogen exchanger 2",
  "gene_symbol": "SLC9A2",
  "term_id": "GO:0015385",
  "gene": "UniProtKB:Q9UBY0"
}